negative regulation of CD8-positive, alpha-beta T cell differentiation [GO:0043377] (biological process) Also known as: down regulation of CD8-positive, alpha-beta T cell differentiation, down-regulation of CD8-positive, alpha-beta T cell differentiation, downregulation of CD8-positive, alpha-beta T cell differentiation, negative regulation of CD8-positive T lymphocyte differentiation, negative regulation of CD8-positive T-cell differentiation, negative regulation of CD8-positive T-lymphocyte differentiation, negative regulation of CD8-positive, alpha beta T lymphocyte differentiation, negative regulation of CD8-positive, alpha beta T-cell differentiation, negative regulation of CD8-positive, alpha beta T-lymphocyte differentiation, inhibition of CD8-positive, alpha-beta T cell differentiation, negative regulation of CD8-positive, alpha-beta T cell development Definition: Any process that stops, prevents, or reduces the rate of CD8-positive, alpha-beta T cell differentiation. Relationships: is a type of regulation of CD8-positive, alpha-beta T cell differentiation [GO:0043376]; is a type of negative regulation of alpha-beta T cell differentiation [GO:0046639]; is a type of negative regulation of CD8-positive, alpha-beta T cell activation [GO:2001186]; RO_0002212 GO:0043374 Sources: GOC:add, ISBN:0781735149 Note: Note that immunologists typically use the word 'development' to refer to cells of B or T cell lineages undergoing the process that GO describes as 'cell differentiation'.